{
  "gene": "UniProtKB:Q5VW22",
  "term_label": "Unknown cellular component",
  "gene_name": "Arf-GAP with GTPase, ANK repeat and PH domain-containing protein 6",
  "term_id": "UNKNOWN:0003",
  "gene_symbol": "AGAP6"
}